regulation of VCP-NPL4-UFD1 AAA ATPase complex assembly [GO:1904239] (biological process) Also known as: regulation of VCP-NPL4-UFD1 AAA ATPase complex formation, regulation of p97-Ufd1-Npl4 complex assembly, regulation of p97-Ufd1-Npl4 complex formation, regulation of Cdc48p-Npl4p-Ufd1p AAA ATPase complex assembly, regulation of Cdc48p-Npl4p-Ufd1p AAA ATPase complex formation Relationships: is a type of regulation of protein-containing complex assembly [GO:0043254]; regulates GO:1904210 Subtypes: GO:1904240, positive regulation of VCP-NPL4-UFD1 AAA ATPase complex assembly [GO:1904241] Definition: Any process that modulates the frequency, rate or extent of VCP-NPL4-UFD1 AAA ATPase complex assembly. Sources: GOC:PARL, GOC:TermGenie, GOC:bf, GO_REF:0000058